{
  "term_label": "Unknown molecular function",
  "term_id": "UNKNOWN:0001",
  "gene_name": "Putative uncharacterized protein FLJ26174",
  "gene": "UniProtKB:Q6ZPA2",
  "gene_symbol": "Q6ZPA2"
}